{
  "gene_name": "Putative uncharacterized protein SNHG12",
  "gene_symbol": "SNHG12",
  "term_label": "Unknown biological process",
  "term_id": "UNKNOWN:0002",
  "gene": "UniProtKB:Q9BXW3"
}